{
  "term_label": "negative regulation of stress fiber assembly",
  "gene": "UniProtKB:Q8IUC4",
  "term_id": "GO:0051497",
  "gene_symbol": "RHPN2",
  "gene_name": "Rhophilin-2"
}